lipid biosynthetic process [GO:0008610] (biological process) Definition: The chemical reactions and pathways resulting in the formation of lipids, compounds soluble in an organic solvent but not, or sparingly, in an aqueous solvent. Relationships: is a type of lipid metabolic process [GO:0006629]; is a type of GO:0009058 Subtypes: fatty acid biosynthetic process [GO:0006633], steroid biosynthetic process [GO:0006694], GO:0008299, GO:0008611, GO:0008654, GO:0009103, glycerolipid biosynthetic process [GO:0045017], neutral lipid biosynthetic process [GO:0046460], GO:0046467, sulfolipid biosynthetic process [GO:0046506], phthiocerol biosynthetic process [GO:0097040], phenolic phthiocerol biosynthetic process [GO:0097041], emericellamide biosynthetic process [GO:1900557], GO:1901570 Also known as: lipid anabolism, lipid biosynthesis, lipid formation, lipid synthesis, lipogenesis Sources: GOC:go_curators Regulation: positively regulated by GO:0046889; regulated by regulation of lipid biosynthetic process [GO:0046890]; negatively regulated by negative regulation of lipid biosynthetic process [GO:0051055]